execution phase of apoptosis [GO:0097194] (biological process) References: PMID:21760595 Sources: GOC:mtg_apoptosis Also known as: execution phase of apoptotic process, apoptosis Definition: A stage of the apoptotic process that starts with the controlled breakdown of the cell through the action of effector caspases or other effector molecules (e.g. cathepsins, calpains etc.). Key steps of the execution phase are rounding-up of the cell, retraction of pseudopodes, reduction of cellular volume (pyknosis), chromatin condensation, nuclear fragmentation (karyorrhexis), plasma membrane blebbing and fragmentation of the cell into apoptotic bodies. When the execution phase is completed, the cell has died. Regulation: regulated by regulation of execution phase of apoptosis [GO:1900117]; negatively regulated by negative regulation of execution phase of apoptosis [GO:1900118]; RO_0002213 by positive regulation of execution phase of apoptosis [GO:1900119] Relationships: is a type of cellular process [GO:0009987]; is part of apoptotic process [GO:0006915]; has part bleb assembly [GO:0032060]